{
  "gene": "UniProtKB:A5PLL1",
  "gene_symbol": "ANKRD34B",
  "term_id": "UNKNOWN:0001",
  "term_label": "Unknown molecular function",
  "gene_name": "Ankyrin repeat domain-containing protein 34B"
}